{
  "gene_symbol": "CARD16",
  "term_label": "Unknown biological process",
  "term_id": "UNKNOWN:0002",
  "gene_name": "Caspase recruitment domain-containing protein 16",
  "gene": "UniProtKB:Q5EG05"
}